{
  "term_label": "endomembrane system",
  "term_id": "GO:0012505",
  "gene_name": "Ras-related protein Rab-21",
  "gene_symbol": "RAB21",
  "gene": "UniProtKB:Q9UL25"
}